{
  "gene_symbol": "SLC32A1",
  "term_label": "dendrite terminus",
  "gene": "UniProtKB:Q9H598",
  "gene_name": "Vesicular inhibitory amino acid transporter",
  "term_id": "GO:0044292"
}